{
  "gene_name": "Homer protein homolog 2",
  "gene": "UniProtKB:Q9NSB8",
  "term_label": "dendrite",
  "gene_symbol": "HOMER2",
  "term_id": "GO:0030425"
}